pyrimidine nucleoside monophosphate catabolic process [GO:0009131] (biological process) Definition: The chemical reactions and pathways resulting in the breakdown of pyrimidine nucleoside monophosphate, a compound consisting of a pyrimidine base linked to a ribose or deoxyribose sugar esterified with phosphate on the sugar. Sources: GOC:go_curators, ISBN:0198506732 Also known as: pyrimidine nucleoside monophosphate breakdown, pyrimidine nucleoside monophosphate catabolism, pyrimidine nucleoside monophosphate degradation Relationships: is_a GO:0009125; is a type of pyrimidine nucleoside monophosphate metabolic process [GO:0009129] Subtypes: GO:0009175, pyrimidine deoxyribonucleoside monophosphate catabolic process [GO:0009178]